{
  "term_id": "GO:0071805",
  "gene": "UniProtKB:Q9H3M0",
  "gene_name": "Potassium voltage-gated channel subfamily F member 1",
  "term_label": "potassium ion transmembrane transport",
  "gene_symbol": "KCNF1"
}